positive regulation of asexual sporulation resulting in formation of a cellular spore [GO:0043945] (biological process) Subtypes: GO:0075249, GO:0075253, GO:0075257, positive regulation of sporangiospore formation [GO:0075287] Sources: GOC:pamgo_curators Definition: Any process that activates, maintains or increases the frequency, rate or extent of the formation of a cellular spore derived from the products of mitosis. Relationships: is a type of GO:0043943; is a type of positive regulation of sporulation resulting in formation of a cellular spore [GO:0045881]; is_a positive regulation of asexual reproduction [GO:1903666]; positively regulates asexual sporulation resulting in formation of a cellular spore [GO:0043936]